{
  "gene_symbol": "DMAC2",
  "gene_name": "Distal membrane-arm assembly complex protein 2",
  "term_id": "GO:0019005",
  "gene": "UniProtKB:Q9NW81",
  "term_label": "SCF ubiquitin ligase complex"
}